nucleotide-excision repair complex [GO:0000109] (cellular component) Note: Note that process information is included in the term and definition for the purpose of describing and distinguishing the complex. Also known as: UvrB-UvrC complex, UvrBC complex Definition: Any complex formed of proteins that act in nucleotide-excision repair. Subtypes: nucleotide-excision repair factor 1 complex [GO:0000110], nucleotide-excision repair factor 2 complex [GO:0000111], nucleotide-excision repair factor 3 complex [GO:0000112], nucleotide-excision repair factor 4 complex [GO:0000113], GO:0070312, ERCC4-ERCC1 complex [GO:0070522], Ddb1-Ckn1 complex [GO:0070912], Ddb1-Wdr21 complex [GO:0070913], GO:0071942 References: PMID:10915862 Relationships: is_a nuclear protein-containing complex [GO:0140513]